{
  "term_label": "Unknown cellular component",
  "gene_symbol": "C4orf50",
  "term_id": "UNKNOWN:0003",
  "gene_name": "Uncharacterized protein C4orf50",
  "gene": "UniProtKB:Q6ZRC1"
}